{
  "term_id": "UNKNOWN:0001",
  "term_label": "Unknown molecular function",
  "gene": "UniProtKB:Q5JU00",
  "gene_name": "Dynein regulatory complex subunit 5",
  "gene_symbol": "TCTE1"
}